{
  "gene": "UniProtKB:Q9BUN5",
  "term_label": "centrosome",
  "term_id": "GO:0005813",
  "gene_symbol": "CCDC28B",
  "gene_name": "Coiled-coil domain-containing protein 28B"
}